{
  "gene": "UniProtKB:Q15058",
  "term_label": "ATP hydrolysis activity",
  "gene_name": "Kinesin-like protein KIF14",
  "gene_symbol": "KIF14",
  "term_id": "GO:0016887"
}